{
  "term_id": "GO:0016887",
  "term_label": "ATP hydrolysis activity",
  "gene_symbol": "KIF3B",
  "gene_name": "Kinesin-like protein KIF3B",
  "gene": "UniProtKB:O15066"
}